{
  "term_label": "serine-type endopeptidase activity",
  "gene": "UniProtKB:P83110",
  "term_id": "GO:0004252",
  "gene_name": "Serine protease HTRA3",
  "gene_symbol": "HTRA3"
}